{
  "term_id": "GO:0016082",
  "gene_symbol": "UNC13A",
  "term_label": "synaptic vesicle priming",
  "gene_name": "Protein unc-13 homolog A",
  "gene": "UniProtKB:Q9UPW8"
}